regulation of transcription by RNA polymerase III [GO:0006359] (biological process) Also known as: regulation of transcription from Pol III promoter, regulation of transcription from RNA polymerase III promoter Subtypes: negative regulation of transcription by RNA polymerase III [GO:0016480], positive regulation of transcription by RNA polymerase III [GO:0045945] Definition: Any process that modulates the frequency, rate or extent of transcription mediated by RNA ploymerase III. Relationships: is a type of regulation of DNA-templated transcription [GO:0006355]; regulates GO:0006383 Sources: GOC:go_curators